retinoic acid metabolic process [GO:0042573] (biological process) Definition: The chemical reactions and pathways involving retinoic acid, one of the three components that makes up vitamin A. References: PMID:12570742 Sources: GOC:jl Also known as: retinoic acid metabolism, vitamin A1 acid metabolic process, vitamin A1 acid metabolism Relationships: is a type of retinoid metabolic process [GO:0001523]; is a type of monocarboxylic acid metabolic process [GO:0032787]; is_a hormone metabolic process [GO:0042445] Subtypes: retinoic acid biosynthetic process [GO:0002138], retinoic acid catabolic process [GO:0034653], 9-cis-retinoic acid metabolic process [GO:0042905]